{
  "term_id": "GO:0005886",
  "gene_symbol": "LYPD5",
  "gene": "UniProtKB:Q6UWN5",
  "gene_name": "Ly6_PLAUR domain-containing protein 5",
  "term_label": "plasma membrane"
}